regulation of pyruvate kinase activity [GO:1903302] (biological process) References: PMID:15804508 Sources: GOC:TermGenie, GOC:mr, GO_REF:0000059 Relationships: is a type of GO:0051338; regulates GO:0004743 Also known as: regulation of ATP:pyruvate 2-O-phosphotransferase activity, regulation of phosphoenol transphosphorylase activity, regulation of phosphoenolpyruvate kinase activity Definition: Any process that modulates the frequency, rate or extent of pyruvate kinase activity.